thyroid-stimulating hormone-secreting cell differentiation [GO:0060129] (biological process) Definition: The process in which a relatively unspecialized cell acquires specialized structural and/or functional features of a thyroid-stimulating hormone-secreting cell. A thyroid-stimulating hormone-secreting cell is a basophil cell of the anterior pituitary that produces thyroid-stimulating hormone, thyrotrophin. Sources: GOC:dph Also known as: TSH-secreting cell differentiation, beta-basophil differentiation, thyroid stimulating hormone secreting cell differentiation, thyrotrope differentiation, thyrotroph differentiation Relationships: is a type of GO:0002067; is a type of GO:0021879; is a type of neuroendocrine cell differentiation [GO:0061101]; is part of adenohypophysis development [GO:0021984]